{
  "term_id": "GO:0006368",
  "term_label": "transcription elongation by RNA polymerase II",
  "gene_name": "Protein polybromo-1",
  "gene_symbol": "PBRM1",
  "gene": "UniProtKB:Q86U86"
}